{
  "gene_name": "Potassium voltage-gated channel subfamily H member 1",
  "term_label": "potassium ion transmembrane transport",
  "term_id": "GO:0071805",
  "gene": "UniProtKB:O95259",
  "gene_symbol": "KCNH1"
}